{
  "gene": "UniProtKB:Q96PC5",
  "gene_name": "Melanoma inhibitory activity protein 2",
  "term_id": "GO:0035459",
  "gene_symbol": "MIA2",
  "term_label": "vesicle cargo loading"
}